{
  "gene_name": "Spermatogenesis-associated protein 2",
  "term_label": "signaling receptor complex adaptor activity",
  "term_id": "GO:0030159",
  "gene_symbol": "SPATA2",
  "gene": "UniProtKB:Q9UM82"
}